extrinsic component of omegasome membrane [GO:0097629] (cellular component) Definition: The component of the omegasome membrane consisting of gene products and protein complexes that are loosely bound to one of its surfaces, but not integrated into the hydrophobic region. Relationships: is a type of GO:0031312; is part of omegasome membrane [GO:1903349] Also known as: extrinsic to omegasome membrane, omegasome peripheral membrane References: PMID:18725538, PMID:24591649 Sources: GOC:mf